endoplasmic reticulum-trans-Golgi network membrane contact site [GO:0160258] (cellular component) Relationships: is a type of organelle membrane contact site [GO:0044232] Definition: An organelle membrane contact site between the endoplasmic reticulum (ER) membrane and the trans-Golgi network (TGN) membrane. References: PMID:30275117, PMID:31732717